primary ureteric bud growth [GO:0060682] (biological process) Definition: The process in which the primary ureteric bud grows along its axis dorsally toward the metanephric blastema. Relationships: is a type of developmental growth involved in morphogenesis [GO:0060560]; is part of ureteric bud elongation [GO:0060677] References: PMID:16916378 Sources: GOC:dph